proteasome core complex, alpha-subunit complex [GO:0019773] (CC) References: PMID:10854779 Sources: GOC:jl, GOC:mtg_sensu, GOC:rb Definition: The proteasome core subcomplex that constitutes the two outer rings of the proteasome core complex. An example of this component is found in Mus musculus. Subtypes: nuclear proteasome core complex, alpha-subunit complex [GO:0031604], cytosolic proteasome core complex, alpha-subunit complex [GO:0031606] Relationships: is a type of protein-containing complex [GO:0032991]; BFO_0000050 intracellular anatomical structure [GO:0005622]; is part of proteasome core complex [GO:0005839]